{
  "gene_symbol": "PLPP7",
  "gene": "UniProtKB:Q8NBV4",
  "term_id": "GO:0005635",
  "term_label": "nuclear envelope",
  "gene_name": "Inactive phospholipid phosphatase 7"
}